{
  "term_label": "Unknown molecular function",
  "gene": "UniProtKB:Q9UBW8",
  "term_id": "UNKNOWN:0001",
  "gene_name": "COP9 signalosome complex subunit 7a",
  "gene_symbol": "COPS7A"
}